cilium or flagellum-dependent cell motility [GO:0001539] (BP) Note: Note that we deem eukaryotic cilia and microtubule-based flagella to be equivalent, while the bacterial- and archaeal-type flagella have a different structure. The former are microtubule-based structures that lash back and forth and are present only in eukaryotes, while the latter achieve motility by rotation. Bacterial- and archaeal-type flagella are superficially similar but have a different molecular composition and fine structure. These three structures never co-exist in the same organism. Therefore, GO:0001539 'cilium or flagellum-dependent cell motility' is in the subset of terms that should not be used for direct gene product annotation. Instead, select a child term. Direct annotations to GO:0001539 'cilium or flagellum-dependent cell motility' may be amended during annotation QC. Sources: GOC:cilia, GOC:hjd, GOC:krc Definition: Cell motility due to movement of eukaryotic cilia or bacterial-type flagella or archaeal-type flagella. Also known as: ciliary/flagellar motility, ciliary or bacterial-type flagellar motility Subtypes: cilium-dependent cell motility [GO:0060285], archaeal or bacterial-type flagellum-dependent cell motility [GO:0097588] Relationships: is a type of cell motility [GO:0048870]